{
  "gene_name": "Immunoglobulin superfamily containing leucine-rich repeat protein",
  "gene_symbol": "ISLR",
  "gene": "UniProtKB:O14498",
  "term_label": "Unknown cellular component",
  "term_id": "UNKNOWN:0003"
}